innervation [GO:0060384] (BP) Definition: The process in which a nerve invades a tissue and makes functional synaptic connection within the tissue. Relationships: is_a GO:0032501; is part of nerve development [GO:0021675] Sources: GOC:dph, GOC:sart